{
  "gene": "UniProtKB:Q9Y328",
  "term_label": "clathrin light chain binding",
  "gene_name": "Neuronal vesicle trafficking-associated protein 2",
  "gene_symbol": "NSG2",
  "term_id": "GO:0032051"
}